{
  "gene": "UniProtKB:Q9H0R6",
  "term_label": "mitochondrion",
  "gene_name": "Glutamyl-tRNA(Gln) amidotransferase subunit A, mitochondrial",
  "term_id": "GO:0005739",
  "gene_symbol": "QRSL1"
}